{
  "gene_name": "Coiled-coil alpha-helical rod protein 1",
  "gene": "UniProtKB:Q8TD31",
  "term_label": "centriole",
  "term_id": "GO:0005814",
  "gene_symbol": "CCHCR1"
}